{
  "term_label": "chromatin binding",
  "gene_symbol": "NCAPH",
  "gene_name": "Condensin complex subunit 2",
  "term_id": "GO:0003682",
  "gene": "UniProtKB:Q15003"
}